leaf vascular tissue pattern formation [GO:0010305] (biological process) Relationships: is a type of xylem and phloem pattern formation [GO:0010051] Definition: Vascular tissue pattern formation as it occurs in the leaf of vascular plants. Sources: GOC:tair_curators